{
  "gene_symbol": "FBRSL1",
  "term_label": "Unknown cellular component",
  "gene_name": "Fibrosin-1-like protein",
  "term_id": "UNKNOWN:0003",
  "gene": "UniProtKB:Q9HCM7"
}